{
  "gene_name": "Carboxypeptidase O",
  "gene": "UniProtKB:Q8IVL8",
  "gene_symbol": "CPO",
  "term_id": "GO:0004181",
  "term_label": "metallocarboxypeptidase activity"
}